{
  "gene_symbol": "RNF17",
  "term_id": "UNKNOWN:0001",
  "term_label": "Unknown molecular function",
  "gene_name": "RING finger protein 17",
  "gene": "UniProtKB:Q9BXT8"
}